{
  "gene_name": "Olfactory receptor 6C65",
  "gene_symbol": "OR6C65",
  "gene": "UniProtKB:A6NJZ3",
  "term_id": "UNKNOWN:0002",
  "term_label": "Unknown biological process"
}